organelle localization [GO:0051640] (biological process) Sources: GOC:ai Subtypes: GO:0033750, GO:0050000, endoplasmic reticulum localization [GO:0051643], plastid localization [GO:0051644], Golgi localization [GO:0051645], mitochondrion localization [GO:0051646], nucleus localization [GO:0051647], vesicle localization [GO:0051648], spindle localization [GO:0051653], GO:0051656, peroxisome localization [GO:0060151], centromere localization [GO:0072765], GO:0140056, vacuolar localization [GO:1990849] Also known as: establishment and maintenance of organelle localization, organelle localisation Relationships: is a type of localization [GO:0051179] Definition: Any process in which an organelle is transported to, and/or maintained in, a specific location.